positive regulation of photoreceptor cell differentiation [GO:0046534] (biological process) Sources: GOC:go_curators Also known as: positive regulation of photoreceptor differentiation, up regulation of photoreceptor cell differentiation, up regulation of photoreceptor differentiation, up-regulation of photoreceptor cell differentiation, up-regulation of photoreceptor differentiation, upregulation of photoreceptor cell differentiation, upregulation of photoreceptor differentiation, activation of photoreceptor cell differentiation, activation of photoreceptor differentiation, stimulation of photoreceptor cell differentiation, stimulation of photoreceptor differentiation Subtypes: positive regulation of eye photoreceptor cell development [GO:0042479], positive regulation of retinal rod cell fate commitment [GO:0060225], positive regulation of compound eye photoreceptor cell differentiation [GO:0110117] Definition: Any process that activates or increases the frequency, rate or extent of photoreceptor cell differentiation. An example of this process is found in Drosophila melanogaster. Relationships: is a type of positive regulation of neuron differentiation [GO:0045666]; is a type of GO:0046532; is a type of positive regulation of multicellular organismal process [GO:0051240]; positively regulates GO:0046530